{
  "term_label": "olfactory receptor activity",
  "gene_name": "Olfactory receptor 10S1",
  "term_id": "GO:0004984",
  "gene": "UniProtKB:Q8NGN2",
  "gene_symbol": "OR10S1"
}